{
  "gene_name": "Ubiquitin carboxyl-terminal hydrolase 10",
  "term_id": "GO:0010506",
  "gene_symbol": "USP10",
  "gene": "UniProtKB:Q14694",
  "term_label": "regulation of autophagy"
}